{
  "gene_symbol": "OR5AC1",
  "term_id": "GO:0004984",
  "gene_name": "Olfactory receptor 5AC1",
  "gene": "UniProtKB:P0C628",
  "term_label": "olfactory receptor activity"
}